{
  "gene": "UniProtKB:P51617",
  "term_label": "Unknown molecular function",
  "gene_symbol": "IRAK1",
  "gene_name": "Interleukin-1 receptor-associated kinase 1",
  "term_id": "UNKNOWN:0001"
}